{
  "gene_symbol": "NOL9",
  "gene": "UniProtKB:Q5SY16",
  "term_id": "GO:0000448",
  "gene_name": "Polynucleotide 5'-hydroxyl-kinase NOL9",
  "term_label": "cleavage in ITS2 between 5.8S rRNA and LSU-rRNA of tricistronic rRNA transcript (SSU-rRNA, 5.8S rRNA, LSU-rRNA)"
}